{
  "term_id": "GO:0043235",
  "term_label": "receptor complex",
  "gene": "UniProtKB:Q9NZD1",
  "gene_symbol": "GPRC5D",
  "gene_name": "G-protein coupled receptor family C group 5 member D"
}